{
  "term_label": "membrane raft",
  "gene_symbol": "CD14",
  "term_id": "GO:0045121",
  "gene": "UniProtKB:P08571",
  "gene_name": "Monocyte differentiation antigen CD14"
}